ABC-type carbohydrate transporter activity [GO:0043211] (molecular function) Relationships: is_a carbohydrate transmembrane transporter activity [GO:0015144]; is a type of ABC-type transporter activity [GO:0140359] Also known as: ATPase-coupled carbohydrate transmembrane transporter activity, ATP-dependent carbohydrate transmembrane transporter activity, carbohydrate-transporting ATPase activity, carbohydrate ABC transporter Subtypes: ABC-type monosaccharide transporter activity [GO:0015407], ABC-type oligosaccharide transporter activity [GO:0015422], ABC-type beta-glucan transporter activity [GO:0015441] Sources: EC:7.5.2.-, GOC:mlg Definition: Enables the transfer of a solute or solutes from one side of a membrane to the other according to the reaction: ATP + H2O = ADP + phosphate, to directly drive the transport of carbohydrates and their derivatives across a membrane.